tobramycin catabolic process [GO:1901120] (biological process) Also known as: tobramycin breakdown, tobramycin catabolism, tobramycin degradation Relationships: is_a glycoside catabolic process [GO:0016139]; is a type of polyol catabolic process [GO:0046174] Sources: GOC:TermGenie, GOC:yaf, UniPathway:UPA00971 Definition: The chemical reactions and pathways resulting in the breakdown of tobramycin.